{
  "term_label": "3',5'-cyclic-AMP phosphodiesterase activity",
  "gene": "UniProtKB:O95263",
  "gene_symbol": "PDE8B",
  "term_id": "GO:0004115",
  "gene_name": "High affinity cAMP-specific and IBMX-insensitive 3',5'-cyclic phosphodiesterase 8B"
}